{
  "gene_symbol": "NINJ1",
  "term_id": "GO:0140912",
  "gene": "UniProtKB:Q92982",
  "term_label": "membrane destabilizing activity",
  "gene_name": "Ninjurin-1"
}